regulation of peptidase activity [GO:0052547] (biological process) Subtypes: negative regulation of peptidase activity [GO:0010466], GO:0010952, regulation of endopeptidase activity [GO:0052548], regulation of metallopeptidase activity [GO:1905048] Sources: GOC:ai Also known as: peptidase regulator activity Relationships: is a type of GO:0030162; is_a regulation of hydrolase activity [GO:0051336]; RO_0002211 peptidase activity [GO:0008233] Definition: Any process that modulates the frequency, rate or extent of peptidase activity, the hydrolysis of peptide bonds within proteins.